{
  "gene_name": "Protoporphyrinogen oxidase",
  "term_id": "GO:0004729",
  "gene": "UniProtKB:P50336",
  "gene_symbol": "PPOX",
  "term_label": "oxygen-dependent protoporphyrinogen oxidase activity"
}